negative regulation of RNA polymerase II regulatory region sequence-specific DNA binding [GO:1903026] (biological process) Definition: Any process that stops, prevents or reduces the frequency, rate or extent of RNA polymerase II regulatory region sequence-specific DNA binding. References: PMID:20026326 Sources: GOC:TermGenie, GOC:dph, GOC:krc, GO_REF:0000059 Also known as: down regulation of RNA polymerase II regulatory region sequence-specific DNA binding, down-regulation of RNA polymerase II regulatory region sequence-specific DNA binding, downregulation of RNA polymerase II regulatory region sequence-specific DNA binding, inhibition of RNA polymerase II regulatory region sequence-specific DNA binding Relationships: is a type of regulation of RNA polymerase II regulatory region sequence-specific DNA binding [GO:1903025]; is a type of negative regulation of transcription regulatory region DNA binding [GO:2000678]; negatively regulates RNA polymerase II transcription regulatory region sequence-specific DNA binding [GO:0000977]